sympathetic neuron projection extension [GO:0097490] (biological process) Definition: Long distance growth of a single sympathetic neuron projection involved in cellular development. A neuron projection is a prolongation or process extending from a nerve cell, e.g. an axon or dendrite. Also known as: sympathetic neuron process extension, sympathetic neuron protrusion extension, sympathetic neuronal cell projection extension, sympathetic neurite extension Relationships: is_a neuron projection extension [GO:1990138] References: PMID:22790009 Sources: GOC:BHF, GOC:rl